{
  "term_id": "GO:0030198",
  "gene": "UniProtKB:Q17RW2",
  "term_label": "extracellular matrix organization",
  "gene_symbol": "COL24A1",
  "gene_name": "Collagen alpha-1(XXIV) chain"
}